{
  "gene": "UniProtKB:Q8IXW0",
  "gene_symbol": "LMNTD2",
  "gene_name": "Lamin tail domain-containing protein 2",
  "term_label": "lamin filament",
  "term_id": "GO:0005638"
}